{
  "gene_name": "PRAME family member 25",
  "gene": "UniProtKB:A6NGN4",
  "gene_symbol": "PRAMEF25",
  "term_label": "cytoplasm",
  "term_id": "GO:0005737"
}